{
  "gene_symbol": "UGT2B10",
  "gene": "UniProtKB:P36537",
  "term_id": "UNKNOWN:0003",
  "gene_name": "UDP-glucuronosyltransferase 2B10",
  "term_label": "Unknown cellular component"
}